{
  "gene": "UniProtKB:P14151",
  "gene_symbol": "SELL",
  "term_id": "GO:0007157",
  "term_label": "heterophilic cell-cell adhesion",
  "gene_name": "L-selectin"
}